{
  "gene_name": "Perforin-1",
  "term_label": "wide pore channel activity",
  "gene_symbol": "PRF1",
  "gene": "UniProtKB:P14222",
  "term_id": "GO:0022829"
}